{
  "term_id": "GO:0051168",
  "gene_name": "Ran-specific GTPase-activating protein",
  "term_label": "nuclear export",
  "gene": "UniProtKB:P43487",
  "gene_symbol": "RANBP1"
}